{
  "gene_name": "Orexin receptor type 2",
  "term_id": "GO:0016499",
  "gene": "UniProtKB:O43614",
  "term_label": "orexin receptor activity",
  "gene_symbol": "HCRTR2"
}